{
  "gene": "UniProtKB:Q5VXH4",
  "gene_symbol": "PRAMEF6",
  "term_id": "GO:0043161",
  "term_label": "proteasome-mediated ubiquitin-dependent protein catabolic process",
  "gene_name": "PRAME family member 6"
}